saccharopine dehydrogenase (NAD+, L-glutamate-forming) activity [GO:0047131] (molecular function) Definition: Catalysis of the reaction: L-saccharopine + H2O + NAD+ = L-glutamate + allysine + H+ + NADH. Also known as: 6-N-(L-1,3-dicarboxypropyl)-L-lysine:NAD+ oxidoreductase (L-glutamate-forming), N6-(L-1,3-dicarboxypropyl)-L-lysine:NAD+ oxidoreductase (L-glutamate-forming), NAD+ oxidoreductase (L-2-aminoadipic-delta-semialdehyde and glutamate forming), aminoadipic semialdehyde synthase activity, dehydrogenase, saccharopine (nicotinamide adenine dinucleotide, glutamate-forming), saccharopin dehydrogenase activity Relationships: is a type of saccharopine dehydrogenase activity [GO:0004753] Sources: EC:1.5.1.9, RHEA:24520